{
  "term_label": "regulation of cellular localization",
  "term_id": "GO:0060341",
  "gene_name": "Partitioning defective 6 homolog alpha",
  "gene": "UniProtKB:Q9NPB6",
  "gene_symbol": "PARD6A"
}